{
  "term_id": "GO:0045944",
  "gene_symbol": "TP53BP1",
  "gene": "UniProtKB:Q12888",
  "gene_name": "TP53-binding protein 1",
  "term_label": "positive regulation of transcription by RNA polymerase II"
}